{
  "term_id": "GO:0038162",
  "gene": "UniProtKB:P19235",
  "gene_name": "Erythropoietin receptor",
  "term_label": "erythropoietin-mediated signaling pathway",
  "gene_symbol": "EPOR"
}